{
  "term_id": "GO:0050767",
  "gene_name": "Hairy and enhancer of split-related protein HELT",
  "gene_symbol": "HELT",
  "term_label": "regulation of neurogenesis",
  "gene": "UniProtKB:A6NFD8"
}